regulation of leaflet formation [GO:0090016] (biological process) Subtypes: positive regulation of leaflet formation by auxin mediated signaling pathway [GO:0090015] Definition: Any process that modulates the frequency, rate or extent of leaflet formation. Relationships: is a type of regulation of leaf morphogenesis [GO:1901371]; regulates GO:0090014 Sources: GOC:dph, GOC:sdb_2009, GOC:tb